{
  "gene": "UniProtKB:Q8NA19",
  "gene_name": "Lethal(3)malignant brain tumor-like protein 4",
  "term_label": "negative regulation of DNA-templated transcription",
  "term_id": "GO:0045892",
  "gene_symbol": "L3MBTL4"
}